{
  "term_label": "cytoskeleton-dependent intracellular transport",
  "gene": "UniProtKB:Q96JE9",
  "gene_name": "Microtubule-associated protein 6",
  "term_id": "GO:0030705",
  "gene_symbol": "MAP6"
}